{
  "gene_symbol": "SLFN14",
  "gene": "UniProtKB:P0C7P3",
  "term_id": "GO:0004521",
  "term_label": "RNA endonuclease activity",
  "gene_name": "Protein SLFN14"
}